{
  "gene_symbol": "C1orf50",
  "term_id": "UNKNOWN:0002",
  "gene_name": "Uncharacterized protein C1orf50",
  "gene": "UniProtKB:Q9BV19",
  "term_label": "Unknown biological process"
}